{
  "gene": "UniProtKB:Q6ZVT0",
  "gene_symbol": "TTLL10",
  "term_id": "UNKNOWN:0003",
  "term_label": "Unknown cellular component",
  "gene_name": "Inactive polyglycylase TTLL10"
}